{
  "term_label": "acrosomal vesicle",
  "gene_symbol": "TCP11X2",
  "gene": "UniProtKB:Q5H9J9",
  "gene_name": "T-complex protein 11 X-linked protein 2",
  "term_id": "GO:0001669"
}